{
  "gene_name": "Reticulophagy regulator 1",
  "term_label": "reticulophagy",
  "gene": "UniProtKB:Q9H6L5",
  "term_id": "GO:0061709",
  "gene_symbol": "RETREG1"
}